{
  "term_label": "nucleus",
  "term_id": "GO:0005634",
  "gene": "UniProtKB:Q6ZNC4",
  "gene_name": "Zinc finger protein 704",
  "gene_symbol": "ZNF704"
}